{
  "term_id": "GO:0033588",
  "gene_name": "Elongator complex protein 2",
  "gene_symbol": "ELP2",
  "gene": "UniProtKB:Q6IA86",
  "term_label": "elongator holoenzyme complex"
}